{
  "gene": "UniProtKB:O60443",
  "gene_name": "Gasdermin-E",
  "term_id": "UNKNOWN:0001",
  "gene_symbol": "GSDME",
  "term_label": "Unknown molecular function"
}